peptide antigen assembly with MHC class II protein complex [GO:0002503] (biological process) References: PMID:15771591 Sources: GOC:add, ISBN:0781735149 Definition: The binding of a peptide to the antigen binding groove of an MHC class II protein complex. Relationships: is a type of peptide antigen assembly with MHC protein complex [GO:0002501]; is part of MHC class II protein complex assembly [GO:0002399]; is part of GO:0002495